{
  "gene": "UniProtKB:A4D1T9",
  "gene_name": "Probable inactive serine protease 37",
  "term_id": "GO:0005615",
  "gene_symbol": "PRSS37",
  "term_label": "extracellular space"
}